{
  "gene_symbol": "SQSTM1",
  "term_label": "K63-linked polyubiquitin modification-dependent protein binding",
  "term_id": "GO:0070530",
  "gene_name": "Sequestosome-1",
  "gene": "UniProtKB:Q13501"
}